{
  "term_id": "GO:0003777",
  "gene": "UniProtKB:Q15058",
  "gene_name": "Kinesin-like protein KIF14",
  "gene_symbol": "KIF14",
  "term_label": "microtubule motor activity"
}